regulation of heart morphogenesis [GO:2000826] (biological process) Sources: GOC:BHF Relationships: is a type of GO:2000027; regulates GO:0003007 Subtypes: heart induction [GO:0003129], regulation of heart induction [GO:0090381], regulation of cardiac chamber morphogenesis [GO:1901219] Definition: Any process that modulates the frequency, rate or extent of heart morphogenesis. Also known as: regulation of cardiac morphogenesis